2,5-dichloro-2,5-cyclohexadiene-1,4-diol dehydrogenase activity [GO:0018502] (molecular function) Relationships: is a type of oxidoreductase activity, acting on the CH-CH group of donors, NAD or NADP as acceptor [GO:0016628] Sources: UM-BBD_reactionID:r0553 Definition: Catalysis of the reaction: 2,5-dichloro-2,5-cyclohexadiene-1,4-diol + NAD+ = NADH + H+ + 2,5-dichlorohydroquinone.